{
  "gene": "UniProtKB:P30626",
  "gene_name": "Sorcin",
  "term_label": "Unknown biological process",
  "term_id": "UNKNOWN:0002",
  "gene_symbol": "SRI"
}